positive regulation of prostaglandin secretion [GO:0032308] (biological process) Sources: GOC:mah Relationships: is a type of positive regulation of icosanoid secretion [GO:0032305]; is a type of regulation of prostaglandin secretion [GO:0032306]; is a type of positive regulation of secretion by cell [GO:1903532]; positively regulates prostaglandin secretion [GO:0032310] Definition: Any process that activates or increases the frequency, rate or extent of the regulated release of a prostaglandin from a cell. Also known as: up regulation of prostaglandin secretion, up-regulation of prostaglandin secretion, upregulation of prostaglandin secretion, activation of prostaglandin secretion, positive regulation of prostacyclin secretion, stimulation of prostaglandin secretion Subtypes: positive regulation of prostaglandin secretion involved in immune response [GO:0061078], positive regulation of fever generation by positive regulation of prostaglandin secretion [GO:0071812]